oxidoreductase activity, acting on the CH-OH group of donors, oxygen as acceptor [GO:0016899] (MF) Definition: Catalysis of an oxidation-reduction (redox) reaction in which a CH-OH group acts as a hydrogen or electron donor and reduces an oxygen molecule. Sources: GOC:ai Relationships: is a type of oxidoreductase activity, acting on CH-OH group of donors [GO:0016614] Subtypes: D-arabinono-1,4-lactone oxidase activity [GO:0003885], (S)-2-hydroxy-acid oxidase activity [GO:0003973], glycerol-3-phosphate oxidase activity [GO:0004369], cholesterol oxidase activity [GO:0016995], GO:0018465, choline:oxygen 1-oxidoreductase activity [GO:0033713], secondary-alcohol oxidase activity [GO:0033714], nucleoside oxidase activity [GO:0033715], GO:0033716, galactose oxidase activity [GO:0045480], GO:0046577, GO:0047579, GO:0047639, GO:0047682, catechol oxidase (dimerizing) activity [GO:0047731], ecdysone oxidase activity [GO:0047875], hexose oxidase activity [GO:0047979], hydroxyphytanate oxidase activity [GO:0047996], L-galactonolactone oxidase activity [GO:0050024], L-sorbose oxidase activity [GO:0050035], L-gulonolactone oxidase activity [GO:0050105], N-acylhexosamine oxidase activity [GO:0050122], polyvinyl-alcohol oxidase activity [GO:0050209], pyranose oxidase activity [GO:0050233], pyridoxine 4-oxidase activity [GO:0050237], thiamine oxidase activity [GO:0050423], GO:0050581, xylitol oxidase activity [GO:0050582], 4-nitrobenzyl alcohol oxidase activity [GO:0102038]